meso-tartrate dehydrogenase activity [GO:0050092] (molecular function) Definition: Catalysis of the reaction: (2R,3S)-tartrate + NAD+ = dihydroxyfumarate + H+ + NADH. Also known as: meso-tartrate:NAD+ oxidoreductase activity Sources: EC:1.3.1.7, RHEA:18553 Relationships: is a type of GO:0016628